{
  "gene_symbol": "NR2C2AP",
  "gene": "UniProtKB:Q86WQ0",
  "gene_name": "Nuclear receptor 2C2-associated protein",
  "term_label": "Unknown molecular function",
  "term_id": "UNKNOWN:0001"
}